{
  "gene": "UniProtKB:P02452",
  "gene_symbol": "COL1A1",
  "term_id": "UNKNOWN:0001",
  "term_label": "Unknown molecular function",
  "gene_name": "Collagen alpha-1(I) chain"
}